{
  "term_id": "GO:0035556",
  "term_label": "intracellular signal transduction",
  "gene_name": "PH domain leucine-rich repeat-containing protein phosphatase 2",
  "gene_symbol": "PHLPP2",
  "gene": "UniProtKB:Q6ZVD8"
}